{
  "term_label": "immune response",
  "gene": "UniProtKB:P10321",
  "term_id": "GO:0006955",
  "gene_name": "HLA class I histocompatibility antigen, C alpha chain",
  "gene_symbol": "HLA-C"
}